{
  "term_id": "GO:0090090",
  "gene": "UniProtKB:Q9UBT3",
  "term_label": "negative regulation of canonical Wnt signaling pathway",
  "gene_name": "Dickkopf-related protein 4",
  "gene_symbol": "DKK4"
}